indole-3-acetic acid amido synthetase activity [GO:0010279] (molecular function) Definition: Catalysis of the reaction: indole-3-acetic acid + an amino acid = an indole-3-acetic acid amide conjugate. References: PMID:15659623 Also known as: IAA amido synthetase activity, IAA amino acid conjugate synthetase activity, IAA amino acid synthetase activity Relationships: is a type of acid-amino acid ligase activity [GO:0016881] Subtypes: GO:0047721